{
  "term_label": "transmembrane transport",
  "term_id": "GO:0055085",
  "gene_symbol": "SLC4A10",
  "gene_name": "Sodium-driven chloride bicarbonate exchanger",
  "gene": "UniProtKB:Q6U841"
}